{
  "gene_name": "Meiosis-specific with OB domain-containing protein",
  "term_id": "UNKNOWN:0003",
  "gene_symbol": "MEIOB",
  "term_label": "Unknown cellular component",
  "gene": "UniProtKB:Q8N635"
}